{
  "term_id": "UNKNOWN:0001",
  "gene_name": "Cell surface glycoprotein MUC18",
  "gene_symbol": "MCAM",
  "term_label": "Unknown molecular function",
  "gene": "UniProtKB:P43121"
}